{
  "term_label": "negative regulation of TOR signaling",
  "gene_name": "Phosphatidylinositol 3,4,5-trisphosphate-dependent Rac exchanger 1 protein",
  "term_id": "GO:0032007",
  "gene_symbol": "PREX1",
  "gene": "UniProtKB:Q8TCU6"
}